{
  "gene": "UniProtKB:Q15785",
  "term_label": "protein targeting to mitochondrion",
  "gene_name": "Mitochondrial import receptor subunit TOM34",
  "gene_symbol": "TOMM34",
  "term_id": "GO:0006626"
}